{
  "gene": "UniProtKB:A6NJY1",
  "term_id": "UNKNOWN:0002",
  "gene_symbol": "SLC9B1P1",
  "gene_name": "Putative SLC9B1-like protein SLC9B1P1",
  "term_label": "Unknown biological process"
}